{
  "term_label": "regulation of synaptic plasticity",
  "gene_symbol": "PLK2",
  "gene_name": "Serine_threonine-protein kinase PLK2",
  "gene": "UniProtKB:Q9NYY3",
  "term_id": "GO:0048167"
}